{
  "gene_symbol": "BAG4",
  "term_id": "GO:0005737",
  "gene": "UniProtKB:O95429",
  "term_label": "cytoplasm",
  "gene_name": "BAG family molecular chaperone regulator 4"
}